{
  "gene": "UniProtKB:O75874",
  "gene_name": "Isocitrate dehydrogenase [NADP] cytoplasmic",
  "term_label": "isocitrate dehydrogenase (NADP+) activity",
  "gene_symbol": "IDH1",
  "term_id": "GO:0004450"
}